{
  "term_label": "serine-type endopeptidase activity",
  "term_id": "GO:0004252",
  "gene_symbol": "GZMH",
  "gene": "UniProtKB:P20718",
  "gene_name": "Granzyme H"
}